mannitol 2-dehydrogenase (NADP+) activity [GO:0050085] (molecular function) Sources: EC:1.1.1.138, RHEA:16765 Definition: Catalysis of the reaction: D-mannitol + NADP+ = D-fructose + H+ + NADPH. Relationships: is_a oxidoreductase activity, acting on the CH-OH group of donors, NAD or NADP as acceptor [GO:0016616] Also known as: D-mannitol:NADP+ 2-oxidoreductase activity, NADP-dependent mannitol dehydrogenase activity